{
  "gene_symbol": "ASH2L",
  "term_label": "Unknown biological process",
  "gene_name": "Set1_Ash2 histone methyltransferase complex subunit ASH2",
  "gene": "UniProtKB:Q9UBL3",
  "term_id": "UNKNOWN:0002"
}